{
  "gene": "UniProtKB:Q14671",
  "term_id": "GO:0005829",
  "term_label": "cytosol",
  "gene_symbol": "PUM1",
  "gene_name": "Pumilio homolog 1"
}